{
  "gene_name": "Eukaryotic translation initiation factor 4E",
  "term_label": "translational initiation",
  "gene_symbol": "EIF4E",
  "gene": "UniProtKB:P06730",
  "term_id": "GO:0006413"
}